{
  "gene_symbol": "A0A6Q8PGZ7",
  "gene": "UniProtKB:A0A6Q8PGZ7",
  "term_id": "UNKNOWN:0003",
  "term_label": "Unknown cellular component",
  "gene_name": "Uncharacterized protein"
}